anther wall tapetum cell differentiation [GO:0048657] (biological process) Also known as: tapetal cell differentiation Definition: The process in which a relatively unspecialized cell acquires specialized features of an anther cell wall tapetum cell. The tapetum is a layer of cells that provides a source of nutrition for the pollen grains as they mature. Sources: GOC:jid, GOC:sm Relationships: is a type of developmental process involved in reproduction [GO:0003006]; is a type of cell differentiation [GO:0030154]; is part of anther wall tapetum formation [GO:0048656]